{
  "gene": "UniProtKB:Q2QL34",
  "term_id": "GO:0005737",
  "term_label": "cytoplasm",
  "gene_symbol": "MPV17L",
  "gene_name": "Mpv17-like protein"
}